urocanate hydratase activity [GO:0016153] (molecular function) Also known as: 3-(5-oxo-4,5-dihydro-3H-imidazol-4-yl)propanoate hydro-lyase (urocanate-forming), 3-(5-oxo-4,5-dihydro-3H-imidazol-4-yl)propanoate hydro-lyase activity, imidazolonepropionate hydrolase activity, urocanase activity Relationships: is_a hydro-lyase activity [GO:0016836] Sources: EC:4.2.1.49, RHEA:13101 Definition: Catalysis of the reaction: 4-imidazolone-5-propanoate + H+ = trans-urocanate + H2O.